{
  "gene": "UniProtKB:B9A6J9",
  "term_id": "UNKNOWN:0003",
  "gene_name": "TBC1 domain family member 3L",
  "term_label": "Unknown cellular component",
  "gene_symbol": "TBC1D3L"
}